oxidoreductase activity, acting on single donors with incorporation of molecular oxygen, incorporation of two atoms of oxygen [GO:0016702] (MF) Sources: GOC:mah Definition: Catalysis of an oxidation-reduction (redox) reaction in which hydrogen or electrons are transferred from one donor, and two oxygen atoms is incorporated into a donor. Relationships: is a type of GO:0016701; is a type of dioxygenase activity [GO:0051213] Subtypes: 3-hydroxyanthranilate 3,4-dioxygenase activity [GO:0000334], beta-carotene 15,15'-dioxygenase activity [GO:0003834], GO:0003868, arachidonate 5-lipoxygenase activity [GO:0004051], arachidonate 12(S)-lipoxygenase activity [GO:0004052], homogentisate 1,2-dioxygenase activity [GO:0004411], L-tryptophan 2,3-dioxygenase activity [GO:0004833], quercetin 2,3-dioxygenase activity [GO:0008127], GO:0008687, acireductone dioxygenase (Ni2+-requiring) activity [GO:0010308], acireductone dioxygenase [iron(II)-requiring] activity [GO:0010309], GO:0010436, linoleate 13S-lipoxygenase activity [GO:0016165], cysteine dioxygenase activity [GO:0017172], p-cumate 2,3-dioxygenase activity [GO:0018570], 2,3-dihydroxy-p-cumate dioxygenase activity [GO:0018571], catechol 1,2-dioxygenase activity [GO:0018576], catechol 2,3-dioxygenase activity [GO:0018577], protocatechuate 3,4-dioxygenase activity [GO:0018578], GO:0018579, hydroxyquinol 1,2-dioxygenase activity [GO:0018581], GO:0018582, biphenyl-2,3-diol 1,2-dioxygenase activity [GO:0018583], acetylacetone-cleaving enzyme activity [GO:0033752], GO:0033754, sulfur oxygenase/reductase activity [GO:0033755], gallate dioxygenase activity [GO:0036238], arachidonate 8(S)-lipoxygenase activity [GO:0036403], GO:0043898, 2,3-dihydroxybenzoate 3,4-dioxygenase activity [GO:0045133], GO:0047069, GO:0047070, 3,4-dihydroxy-9,10-secoandrosta-1,3,5(10)-triene-9,17-dione 4,5-dioxygenase activity [GO:0047071], 2,3-dihydroxybenzoate 2,3-dioxygenase activity [GO:0047072], 2,4'-dihydroxyacetophenone dioxygenase activity [GO:0047073], GO:0047074, GO:0047075, 3-hydroxy-4-oxoquinoline 2,4-dioxygenase activity [GO:0047078], 2,3-dihydroxyindole 2,3-dioxygenase activity [GO:0047528], arachidonate 8(R)-lipoxygenase activity [GO:0047677], GO:0047719, chloridazon-catechol dioxygenase activity [GO:0047744], caffeate 3,4-dioxygenase activity [GO:0047762], cysteamine dioxygenase activity [GO:0047800], gentisate 1,2-dioxygenase activity [GO:0047922], GO:0050054, pyrogallol 1,2-oxygenase activity [GO:0050240], stizolobate synthase activity [GO:0050297], GO:0050298, sulfur dioxygenase activity [GO:0050313], arachidonate 15-lipoxygenase activity [GO:0050473], GO:0050584, GO:0050585, 3-hydroxy-2-methylquinolin-4-one 2,4-dioxygenase activity [GO:0050586], chlorite O2-lyase activity [GO:0050587], linoleate 8R-lipoxygenase activity [GO:0052878], beta,beta-carotene-9',10'-cleaving oxygenase activity [GO:0102076], all-trans-8'-apo-beta-carotenal 15,15'-oxygenase activity [GO:0102162], all-trans-beta-apo-10'-carotenal cleavage oxygenase activity [GO:0102251], linolenate 9R-lipoxygenase activity [GO:0102299], 9-cis-beta-carotene 9',10'-cleavage oxygenase activity [GO:0102395], 9-cis-10'-apo-beta-carotenal cleavage oxygenase activity [GO:0102396], fatty acid alpha-dioxygenase activity [GO:0102672], GO:0102785, 5,6-dimethylbenzimidazole synthase activity [GO:0102919], arachidonate 12(R)-lipoxygenase activity [GO:0106237], linoleate 9S-lipoxygenase activity [GO:1990136]